positive regulation of cristae formation [GO:1903852] (biological process) Definition: Any process that activates or increases the frequency, rate or extent of cristae formation. References: PMID:19279012 Sources: GOC:PARL, GOC:TermGenie, GOC:pad, GO_REF:0000058 Also known as: up regulation of cristae formation, up-regulation of cristae formation, upregulation of cristae formation, activation of cristae formation Note: AN example of this is PINK1 in human (Q9BXM7) in PMID:19279012 inferred from mutant phenotype Relationships: is a type of positive regulation of organelle organization [GO:0010638]; is a type of GO:1903850; positively regulates cristae formation [GO:0042407]